response to olanzapine [GO:0097333] (biological process) Definition: Any process that results in a change in state or activity of a cell or an organism (in terms of movement, secretion, enzyme production, gene expression, etc.) as a result of an olanzapine stimulus. Sources: GOC:pr Relationships: is a type of GO:1901698